B cell mediated immunity [GO:0019724] (biological process) Relationships: is a type of lymphocyte mediated immunity [GO:0002449]; is a type of GO:0002460 Subtypes: GO:0002368, peripheral B cell tolerance induction [GO:0002451], immunoglobulin mediated immune response [GO:0016064] Also known as: B lymphocyte mediated immune effector process, B lymphocyte mediated immunity, B-cell mediated immune effector process, B-cell mediated immunity, B-lymphocyte mediated immune effector process, B-lymphocyte mediated immunity Regulation: regulated by regulation of B cell mediated immunity [GO:0002712]; negatively regulated by GO:0002713; positively regulated by positive regulation of B cell mediated immunity [GO:0002714] Sources: GOC:add, GO_REF:0000022, ISBN:0781735149 Definition: Any process involved with the carrying out of an immune response by a B cell, through, for instance, the production of antibodies or cytokines, or antigen presentation to T cells.